{
  "term_label": "Unknown biological process",
  "term_id": "UNKNOWN:0002",
  "gene": "UniProtKB:A6NJQ4",
  "gene_name": "Putative protein FAM90A8",
  "gene_symbol": "FAM90A8"
}